microsporidian-type endospore [GO:0090641] (cellular component) Definition: The middle layer in a microsporidian spore wall that lies under the exospore and outside the plasma membrane, containing chitin and proteins. References: PMID:19457051 Note: Microsporidian biology uses the term endospore differently than GO:0043593 endospore coat which is for a spore formed inside of another cell. Microsporidian endospore refers to the inner layer of the spore wall itself. Relationships: is a type of cellular anatomical structure [GO:0110165]; is part of spore wall [GO:0031160]